positive regulation of immature T cell proliferation in thymus [GO:0033092] (BP) Relationships: is a type of regulation of immature T cell proliferation in thymus [GO:0033084]; is a type of GO:0033091; positively regulates GO:0033080 Also known as: positive regulation of thymic T cell proliferation, positive regulation of thymocyte cell proliferation, positive regulation of thymocyte proliferation Sources: GOC:add, GOC:mah Definition: Any process that activates or increases the frequency, rate or extent of immature T cell proliferation in the thymus.